{
  "term_label": "cytoplasm",
  "gene": "UniProtKB:Q9NXD2",
  "gene_symbol": "MTMR10",
  "term_id": "GO:0005737",
  "gene_name": "Myotubularin-related protein 10"
}